{
  "gene_symbol": "ASGR2",
  "gene_name": "Asialoglycoprotein receptor 2",
  "gene": "UniProtKB:P07307",
  "term_id": "GO:0005537",
  "term_label": "D-mannose binding"
}